{
  "gene_symbol": "PCDHA8",
  "gene_name": "Protocadherin alpha-8",
  "term_id": "GO:0007155",
  "gene": "UniProtKB:Q9Y5H6",
  "term_label": "cell adhesion"
}